regulation of action potential firing threshold [GO:0099611] (BP) Sources: ISBN:978-0071390118 Relationships: is_a GO:0098900 Definition: Any process that regulates the potential at which an axon potential is triggered.